gap junction channel activity involved in SA node cell-atrial cardiac muscle cell electrical coupling [GO:0086020] (molecular function) Relationships: is_a GO:0086075; is part of SA node cell to atrial cardiac muscle cell communication by electrical coupling [GO:0086021] Sources: GOC:BHF, GOC:mtg_cardiac_conduct_nov11 Definition: A wide pore channel activity that enables a direct cytoplasmic connection from an SA node cell to an atrial cardiomyocyte. The gap junction passes electrical signals between the cells contributing to cardiac conduction. Also known as: gap junction channel activity involved in SA node cell-atrial cardiomyocyte electrical coupling, gap junction channel activity involved in SAN cell-atrial cardiomyocyte electrical coupling, gap junction channel activity involved in sinoatrial node cell-atrial cardiomyocyte electrical coupling, gap junction channel activity involved in sinus node cell-atrial cardiomyocyte electrical coupling